{
  "term_id": "GO:0005654",
  "gene_symbol": "IFI16",
  "gene": "UniProtKB:Q16666",
  "term_label": "nucleoplasm",
  "gene_name": "Gamma-interferon-inducible protein 16"
}